neutrophil-mediated killing of symbiont cell [GO:0070943] (biological process) Regulation: regulated by regulation of neutrophil mediated killing of symbiont cell [GO:0070949]; negatively regulated by negative regulation of neutrophil mediated killing of symbiont cell [GO:0070955]; positively regulated by positive regulation of neutrophil mediated killing of symbiont cell [GO:0070961] Also known as: neutrophil mediated killing of symbiont cell Subtypes: GO:0070944, neutrophil-mediated killing of fungus [GO:0070947] Sources: GOC:add, ISBN:0781765196 Definition: The directed killing of a symbiont target cell by a neutrophil. The symbiont is defined as the smaller of the organisms involved in a symbiotic interaction. Relationships: is a type of killing by host of symbiont cells [GO:0051873]; is a type of neutrophil mediated cytotoxicity [GO:0070942]